{
  "gene_name": "Nesprin-2",
  "term_id": "GO:1902017",
  "gene_symbol": "SYNE2",
  "term_label": "regulation of cilium assembly",
  "gene": "UniProtKB:Q8WXH0"
}